{
  "term_id": "GO:0051015",
  "gene_name": "Huntingtin-interacting protein 1",
  "term_label": "actin filament binding",
  "gene_symbol": "HIP1",
  "gene": "UniProtKB:O00291"
}